{
  "gene": "UniProtKB:Q9BRZ2",
  "term_label": "nucleoplasm",
  "gene_name": "E3 ubiquitin-protein ligase TRIM56",
  "term_id": "GO:0005654",
  "gene_symbol": "TRIM56"
}